{
  "term_id": "UNKNOWN:0001",
  "gene_name": "Serine-rich and transmembrane domain-containing 2",
  "term_label": "Unknown molecular function",
  "gene": "UniProtKB:A0A1B0GWG4",
  "gene_symbol": "SERTM2"
}